acylpyruvate hydrolase activity [GO:0047621] (molecular function) Sources: RHEA:19009 Relationships: is a type of hydrolase activity, acting on acid carbon-carbon bonds, in ketonic substances [GO:0016823] Definition: Catalysis of the reaction: a 3-acylpyruvate + H2O = a carboxylate + pyruvate. Also known as: 3-acylpyruvate acylhydrolase activity